{
  "term_label": "Unknown molecular function",
  "gene": "UniProtKB:A0A075B6L6",
  "gene_symbol": "TRBV7-3",
  "gene_name": "Probable non-functional T cell receptor beta variable 7-3",
  "term_id": "UNKNOWN:0001"
}